intracellular nucleoside homeostasis [GO:0140980] (biological process) Relationships: is a type of intracellular chemical homeostasis [GO:0055082] References: PMID:23416111, PMID:34880500 Definition: A homeostatic process involved in the maintenance of a steady state level of nucleosides within a cell.